{
  "term_label": "Unknown biological process",
  "term_id": "UNKNOWN:0002",
  "gene_symbol": "GSTCD",
  "gene_name": "Glutathione S-transferase C-terminal domain-containing protein",
  "gene": "UniProtKB:Q8NEC7"
}